{
  "gene_symbol": "ZNF106",
  "term_label": "cytosol",
  "gene_name": "Zinc finger protein 106",
  "term_id": "GO:0005829",
  "gene": "UniProtKB:Q9H2Y7"
}